{
  "gene_symbol": "TLCD5",
  "gene_name": "TLC domain-containing protein 5",
  "term_label": "Unknown molecular function",
  "gene": "UniProtKB:Q6ZRR5",
  "term_id": "UNKNOWN:0001"
}